regulation of methanophenazine biosynthetic process [GO:1900962] (biological process) Subtypes: GO:1900963, positive regulation of methanophenazine biosynthetic process [GO:1900964] Sources: GOC:TermGenie, GOC:mengo_curators Also known as: regulation of methanophenazine anabolism, regulation of methanophenazine biosynthesis, regulation of methanophenazine formation, regulation of methanophenazine synthesis Relationships: is a type of regulation of biosynthetic process [GO:0009889]; regulates methanophenazine biosynthetic process [GO:1900630] Definition: Any process that modulates the frequency, rate or extent of methanophenazine biosynthetic process.